{
  "term_id": "UNKNOWN:0001",
  "gene": "UniProtKB:Q8N0T1",
  "term_label": "Unknown molecular function",
  "gene_name": "Ribosomal biogenesis factor",
  "gene_symbol": "RBIS"
}